{
  "gene_symbol": "WDFY3",
  "gene": "UniProtKB:Q8IZQ1",
  "term_label": "aggrephagy",
  "term_id": "GO:0035973",
  "gene_name": "WD repeat and FYVE domain-containing protein 3"
}